neuropeptide activity [GO:0160041] (molecular function) Relationships: is a type of receptor ligand activity [GO:0048018]; has part neuropeptide receptor binding [GO:0071855] References: PMID:18806786, PMID:21922398 Definition: The receptor ligand activity of any polypeptide expressed in, and secreted from a neuron. Subtypes: GO:0005184